negative regulation of dense core granule biogenesis [GO:2000706] (biological process) Sources: GOC:obol Definition: Any process that stops, prevents or reduces the frequency, rate or extent of dense core granule biogenesis. Relationships: is a type of negative regulation of cellular process [GO:0048523]; is a type of regulation of dense core granule biogenesis [GO:2000705]; negatively regulates GO:0061110